{
  "term_label": "Unknown biological process",
  "gene": "UniProtKB:O95395",
  "gene_name": "Beta-1,3-galactosyl-O-glycosyl-glycoprotein beta-1,6-N-acetylglucosaminyltransferase 3",
  "term_id": "UNKNOWN:0002",
  "gene_symbol": "GCNT3"
}